{
  "term_label": "Unknown cellular component",
  "gene": "UniProtKB:O60543",
  "term_id": "UNKNOWN:0003",
  "gene_name": "Lipid transferase CIDEA",
  "gene_symbol": "CIDEA"
}